ligase activity, forming carbon-sulfur bonds [GO:0016877] (molecular function) Sources: EC:6.2.-.- Subtypes: ubiquitin-like modifier activating enzyme activity [GO:0008641], CoA-ligase activity [GO:0016405], GO:0016878 Relationships: is a type of GO:0016874 Definition: Catalysis of the joining of two molecules via a carbon-sulfur bond, with the concomitant hydrolysis of the diphosphate bond in ATP or a similar triphosphate. Also known as: ligase activity, forming carbon-sulphur bonds